glucosamine-containing compound catabolic process [GO:1901072] (biological process) Definition: The chemical reactions and pathways resulting in the breakdown of glucosamine-containing compounds (glucosamines). Relationships: is a type of amino sugar catabolic process [GO:0046348] Subtypes: chitin catabolic process [GO:0006032], glucosamine catabolic process [GO:0006043], N-acetylglucosamine catabolic process [GO:0006046] Also known as: glucosamine-containing compound breakdown, glucosamine-containing compound catabolism, glucosamine-containing compound degradation, glucosamines breakdown, glucosamines catabolic process, glucosamines catabolism, glucosamines degradation Sources: GOC:TermGenie